{
  "gene_name": "Dual oxidase 1",
  "gene_symbol": "DUOX1",
  "term_id": "GO:0005886",
  "term_label": "plasma membrane",
  "gene": "UniProtKB:Q9NRD9"
}